{
  "term_id": "UNKNOWN:0002",
  "gene_name": "Serpin B8",
  "term_label": "Unknown biological process",
  "gene": "UniProtKB:P50452",
  "gene_symbol": "SERPINB8"
}